{
  "term_id": "GO:0031012",
  "gene_name": "Microfibril-associated glycoprotein 4",
  "gene": "UniProtKB:P55083",
  "gene_symbol": "MFAP4",
  "term_label": "extracellular matrix"
}